{
  "gene_name": "Hairy_enhancer-of-split related with YRPW motif-like protein",
  "term_label": "RNA polymerase II cis-regulatory region sequence-specific DNA binding",
  "gene_symbol": "HEYL",
  "term_id": "GO:0000978",
  "gene": "UniProtKB:Q9NQ87"
}